DNA import into cell involved in transformation [GO:0009290] (biological process) Also known as: DNA import into cell, cellular DNA uptake, DNA transport into cell during transformation, cellular DNA import during transformation Relationships: is a type of DNA transport [GO:0051027]; is_a GO:0098657; is part of GO:0009294 Sources: GOC:ai Definition: The directed movement of DNA into a cell that contributes to the process of transformation, the uptake of foreign genetic material into a cell.